{
  "gene_name": "SUN domain-containing protein 1",
  "gene": "UniProtKB:O94901",
  "gene_symbol": "SUN1",
  "term_label": "protein-membrane adaptor activity",
  "term_id": "GO:0043495"
}